{
  "gene_symbol": "VBP1",
  "gene": "UniProtKB:P61758",
  "term_id": "GO:0007021",
  "gene_name": "Prefoldin subunit 3",
  "term_label": "tubulin complex assembly"
}